{
  "term_id": "GO:0016601",
  "gene_symbol": "NISCH",
  "gene_name": "Nischarin",
  "gene": "UniProtKB:Q9Y2I1",
  "term_label": "Rac protein signal transduction"
}